type B pancreatic cell proliferation [GO:0044342] (biological process) Sources: GOC:jl, GOC:yaf Definition: The multiplication or reproduction of pancreatic B cells, resulting in the expansion of an pancreatic B cell population. Pancreatic B cell are cells of the pancreas that secrete insulin. Relationships: is a type of epithelial cell proliferation [GO:0050673] Regulation: regulated by regulation of type B pancreatic cell proliferation [GO:0061469]; negatively regulated by negative regulation of type B pancreatic cell proliferation [GO:1904691]; positively regulated by positive regulation of type B pancreatic cell proliferation [GO:1904692] Also known as: pancreatic B cell proliferation, pancreatic beta cell proliferation